{
  "term_label": "mRNA binding",
  "gene": "UniProtKB:P62995",
  "gene_symbol": "TRA2B",
  "term_id": "GO:0003729",
  "gene_name": "Transformer-2 protein homolog beta"
}